seminiferous tubule development [GO:0072520] (biological process) Relationships: is a type of tube development [GO:0035295]; is a type of GO:0048608; is part of GO:0008584 Sources: GOC:BHF, GOC:mah, UBERON:0001343 Definition: The reproductive developmental process whose specific outcome is the progression of the seminiferous tubule over time, from its formation to the mature structure. Seminiferous tubules are ducts located in the testicles, and are the specific location of meiosis, and the subsequent creation of gametes, namely spermatozoa.